{
  "gene_name": "Arachidonate 5-lipoxygenase-activating protein",
  "gene": "UniProtKB:P20292",
  "gene_symbol": "ALOX5AP",
  "term_label": "nuclear envelope",
  "term_id": "GO:0005635"
}